telomeric DNA-containing double minutes formation [GO:0061819] (biological process) References: PMID:14690602, PMID:2397458 Sources: GOC:BHF, GOC:BHF_telomere, GOC:nc Definition: A telomere maintenance process that results in the formation of small fragments of circular extrachromosomal DNA elements which contain telomeric DNA. It is speculated that telomeric DNA-containing double minutes are formed through a recombination event between the telomere and chromosome-internal TTAGGG-like sequences. Telomeric DNA-containing double minutes appear as two closely positioned dots in metaphase. Relationships: is_a telomere maintenance via recombination [GO:0000722] Also known as: TDMs formation